{
  "gene_name": "Olfactory receptor 8H1",
  "term_label": "G protein-coupled receptor signaling pathway",
  "term_id": "GO:0007186",
  "gene": "UniProtKB:Q8NGG4",
  "gene_symbol": "OR8H1"
}